{
  "gene": "UniProtKB:A2RU67",
  "term_label": "Unknown biological process",
  "gene_symbol": "FAM234B",
  "gene_name": "Protein FAM234B",
  "term_id": "UNKNOWN:0002"
}